{
  "term_id": "GO:0006357",
  "gene_name": "Rhox homeobox family member 2B",
  "gene_symbol": "RHOXF2B",
  "gene": "UniProtKB:P0C7M4",
  "term_label": "regulation of transcription by RNA polymerase II"
}